negative regulation of defense response [GO:0031348] (biological process) Also known as: down regulation of defense response, down-regulation of defense response, downregulation of defense response, inhibition of defense response Relationships: is a type of regulation of defense response [GO:0031347]; is a type of negative regulation of response to stimulus [GO:0048585]; negatively regulates defense response [GO:0006952] Sources: GOC:mah Subtypes: negative regulation of antimicrobial humoral response [GO:0008348], GO:0010113, negative regulation of innate immune response [GO:0045824], GO:0050687, negative regulation of inflammatory response [GO:0050728], GO:0051245, negative regulation of neutrophil mediated killing of symbiont cell [GO:0070955], negative regulation of defense response to insect [GO:1900366], GO:1900425, GO:1902289, negative regulation of xenophagy [GO:1904416], negative regulation of behavioral fear response [GO:2000986] Definition: Any process that stops, prevents, or reduces the frequency, rate or extent of a defense response.